{
  "gene": "UniProtKB:P35243",
  "term_id": "UNKNOWN:0003",
  "gene_name": "Recoverin",
  "gene_symbol": "RCVRN",
  "term_label": "Unknown cellular component"
}